mast cell proliferation [GO:0070662] (biological process) Relationships: is a type of leukocyte proliferation [GO:0070661] Regulation: regulated by GO:0070666; negatively regulated by GO:0070667; positively regulated by positive regulation of mast cell proliferation [GO:0070668] Sources: GOC:add Definition: The expansion of a mast cell population by cell division.